{
  "gene_symbol": "ESCO2",
  "gene": "UniProtKB:Q56NI9",
  "gene_name": "N-acetyltransferase ESCO2",
  "term_id": "GO:0005634",
  "term_label": "nucleus"
}